{
  "term_id": "GO:0034765",
  "term_label": "regulation of monoatomic ion transmembrane transport",
  "gene_name": "NEDD4-like E3 ubiquitin-protein ligase WWP2",
  "gene": "UniProtKB:O00308",
  "gene_symbol": "WWP2"
}